{
  "gene": "UniProtKB:Q96A98",
  "gene_name": "Tuberoinfundibular peptide of 39 residues",
  "gene_symbol": "PTH2",
  "term_id": "UNKNOWN:0003",
  "term_label": "Unknown cellular component"
}